{
  "term_id": "UNKNOWN:0001",
  "gene_name": "Secretoglobin family 1C member 1",
  "gene": "UniProtKB:Q8TD33",
  "term_label": "Unknown molecular function",
  "gene_symbol": "SCGB1C1"
}